{
  "gene": "UniProtKB:P43354",
  "gene_symbol": "NR4A2",
  "term_label": "transcription regulator complex",
  "term_id": "GO:0005667",
  "gene_name": "Nuclear receptor subfamily 4 group A member 2"
}